tyrosine transport [GO:0015828] (biological process) Definition: The directed movement of tyrosine, 2-amino-3-(4-hydroxyphenyl)propanoic acid, into, out of or within a cell, or between cells, by means of some agent such as a transporter or pore. Sources: GOC:ai Subtypes: L-tyrosine transmembrane import into vacuole [GO:0090514], L-tyrosine import across plasma membrane [GO:1903808] Relationships: is a type of organic cation transport [GO:0015695]; is a type of aromatic amino acid transport [GO:0015801]; is a type of L-amino acid transport [GO:0015807] Also known as: L-tyrosine transport